tryprostatin A biosynthetic process [GO:0140654] (biological process) Relationships: is a type of indole alkaloid biosynthetic process [GO:0035835]; is a type of indole-containing compound biosynthetic process [GO:0042435]; is a type of amide biosynthetic process [GO:0043604]; is a type of ether biosynthetic process [GO:1901503] Definition: The chemical reactions and pathways resulting in the formation of tryprostatin A. References: PMID:19226505 Sources: GOC:ach Also known as: tryprostatin A anabolism, tryprostatin A biosynthesis, tryprostatin A formation, tryprostatin A synthesis